{
  "term_label": "regulation of immune system process",
  "gene_name": "B-cell lymphoma 6 protein",
  "term_id": "GO:0002682",
  "gene": "UniProtKB:P41182",
  "gene_symbol": "BCL6"
}